{
  "gene_name": "Testis-expressed protein 52",
  "term_label": "Unknown molecular function",
  "gene": "UniProtKB:A6NCN8",
  "term_id": "UNKNOWN:0001",
  "gene_symbol": "TEX52"
}